{
  "term_id": "GO:0006511",
  "gene_name": "Ubiquitin-like protein 7",
  "gene_symbol": "UBL7",
  "term_label": "ubiquitin-dependent protein catabolic process",
  "gene": "UniProtKB:Q96S82"
}